{
  "term_id": "GO:0035005",
  "term_label": "1-phosphatidylinositol-4-phosphate 3-kinase activity",
  "gene_symbol": "PIK3CG",
  "gene_name": "Phosphatidylinositol 4,5-bisphosphate 3-kinase catalytic subunit gamma isoform",
  "gene": "UniProtKB:P48736"
}